positive regulation of neutrophil mediated killing of bacterium [GO:0070962] (biological process) Sources: GOC:add, GOC:mah Definition: Any process that increases the frequency, rate or extent of the directed killing of a bacterium by a neutrophil. Relationships: is a type of GO:0070950; is a type of GO:0070961; is a type of positive regulation of defense response to bacterium [GO:1900426]; positively regulates neutrophil-mediated killing of bacterium [GO:0070944] Also known as: up regulation of neutrophil mediated killing of bacterium, up-regulation of neutrophil mediated killing of bacterium, upregulation of neutrophil mediated killing of bacterium, activation of neutrophil mediated killing of bacterium, stimulation of neutrophil mediated killing of bacterium Subtypes: positive regulation of neutrophil mediated killing of gram-negative bacterium [GO:0070963], GO:0070964